Spemann organizer formation [GO:0060061] (biological process) Definition: Formation of the specialized region on the dorsalmost side of the embryo that acts as the main signaling center establishing the vertebrate body plan. Subtypes: Spemann organizer formation at the dorsal lip of the blastopore [GO:0060062], Spemann organizer formation at the embryonic shield [GO:0060063], Spemann organizer formation at the anterior end of the primitive streak [GO:0060064] Sources: GOC:bf, GOC:dph Also known as: Spemann's organizer formation, Spemann-Mangold organizer formation Relationships: is a type of GO:0048646; is part of GO:0031128